{
  "gene_name": "Receptor-transporting protein 1",
  "gene": "UniProtKB:P59025",
  "term_id": "GO:0009986",
  "term_label": "cell surface",
  "gene_symbol": "RTP1"
}